{
  "gene": "UniProtKB:Q9Y4C0",
  "gene_name": "Neurexin-3",
  "term_label": "trans-synaptic protein complex",
  "term_id": "GO:0098820",
  "gene_symbol": "NRXN3"
}